{
  "term_label": "Unknown biological process",
  "gene": "UniProtKB:Q8N2H3",
  "gene_name": "Pyridine nucleotide-disulfide oxidoreductase domain-containing protein 2",
  "term_id": "UNKNOWN:0002",
  "gene_symbol": "PYROXD2"
}